{
  "gene_name": "Actin filament-associated protein 1-like 2",
  "gene": "UniProtKB:Q8N4X5",
  "gene_symbol": "AFAP1L2",
  "term_id": "GO:0045893",
  "term_label": "positive regulation of DNA-templated transcription"
}